{
  "gene": "UniProtKB:Q13445",
  "term_id": "GO:0005783",
  "gene_name": "Transmembrane emp24 domain-containing protein 1",
  "gene_symbol": "TMED1",
  "term_label": "endoplasmic reticulum"
}